IAA-Leu conjugate hydrolase activity [GO:0010211] (molecular function) Definition: Catalysis of the reaction: indole-3-acetyl-leucine + H2O = indole-3-acetate + L-leucine. Sources: MetaCyc:RXN-2982 Relationships: is_a IAA-amino acid conjugate hydrolase activity [GO:0010178]